cellular response to oxidopamine [GO:1905842] (BP) References: PMID:23721876 Sources: GOC:TermGenie, GOC:rz, GO_REF:0000071 Regulation: regulated by regulation of cellular response to oxidopamine [GO:1905846]; negatively regulated by GO:1905847; positively regulated by positive regulation of cellular response to oxidopamine [GO:1905848] Relationships: is a type of cellular response to catecholamine stimulus [GO:0071870]; is_a response to oxidopamine [GO:1905841] Definition: Any process that results in a change in state or activity of a cell (in terms of movement, secretion, enzyme production, gene expression, etc.) as a result of an oxidopamine stimulus.